{
  "gene_symbol": "GTF2H5",
  "gene": "UniProtKB:Q6ZYL4",
  "term_label": "transcription factor TFIIH holo complex",
  "gene_name": "General transcription factor IIH subunit 5",
  "term_id": "GO:0005675"
}